ribosome [GO:0005840] (cellular component) Relationships: is a type of intracellular membraneless organelle [GO:0043232] Sources: ISBN:0198506732 Also known as: free ribosome, membrane bound ribosome, ribosomal RNA Subtypes: organellar ribosome [GO:0000313], cytosolic ribosome [GO:0022626] Definition: An intracellular organelle, about 200 A in diameter, consisting of RNA and protein. It is the site of protein biosynthesis resulting from translation of messenger RNA (mRNA). It consists of two subunits, one large and one small, each containing only protein and RNA. Both the ribosome and its subunits are characterized by their sedimentation coefficients, expressed in Svedberg units (symbol: S). Hence, the prokaryotic ribosome (70S) comprises a large (50S) subunit and a small (30S) subunit, while the eukaryotic ribosome (80S) comprises a large (60S) subunit and a small (40S) subunit. Two sites on the ribosomal large subunit are involved in translation, namely the aminoacyl site (A site) and peptidyl site (P site). Ribosomes from prokaryotes, eukaryotes, mitochondria, and chloroplasts have characteristically distinct ribosomal proteins.